{
  "term_label": "Unknown molecular function",
  "gene_symbol": "TBRG1",
  "gene_name": "Transforming growth factor beta regulator 1",
  "term_id": "UNKNOWN:0001",
  "gene": "UniProtKB:Q3YBR2"
}